{
  "gene_symbol": "GPR18",
  "gene_name": "N-arachidonyl glycine receptor",
  "term_id": "GO:0007186",
  "gene": "UniProtKB:Q14330",
  "term_label": "G protein-coupled receptor signaling pathway"
}